{
  "term_id": "UNKNOWN:0003",
  "gene_name": "NUT family member 2G",
  "gene_symbol": "NUTM2G",
  "gene": "UniProtKB:Q5VZR2",
  "term_label": "Unknown cellular component"
}